{
  "gene": "UniProtKB:Q99453",
  "term_label": "enteric nervous system development",
  "gene_symbol": "PHOX2B",
  "gene_name": "Paired mesoderm homeobox protein 2B",
  "term_id": "GO:0048484"
}